regulation of iron ion transmembrane transport [GO:0034759] (biological process) Definition: Any process that modulates the frequency, rate or extent of the directed movement of iron ions (Fe) from one side of a membrane to the other by means of some agent such as a transporter or pore. Also known as: regulation of iron ion membrane transport, regulation of transmembrane Fe transport, regulation of transmembrane iron ion transport, regulation of transmembrane iron transport Relationships: is_a regulation of iron ion transport [GO:0034756]; is a type of regulation of monoatomic cation transmembrane transport [GO:1904062]; regulates iron ion transmembrane transport [GO:0034755] Sources: GOC:mah Subtypes: GO:0034760, GO:0034761, regulation of iron export across plasma membrane [GO:1904038], regulation of iron ion import across plasma membrane [GO:1904438]